negative regulation of protein localization to cell tip [GO:1903067] (biological process) References: PMID:24554432 Sources: GOC:TermGenie, GO_REF:0000058 Relationships: is a type of regulation of protein localization to cell tip [GO:1903066]; is a type of negative regulation of protein localization [GO:1903828]; negatively regulates protein localization to cell tip [GO:1990151] Subtypes: GO:0062108 Definition: Any process that stops, prevents or reduces the frequency, rate or extent of protein localization to cell tip. Also known as: down regulation of protein localisation to cell tip, down regulation of protein localization to cell tip, down-regulation of protein localisation to cell tip, down-regulation of protein localization to cell tip, downregulation of protein localisation to cell tip, downregulation of protein localization to cell tip, negative regulation of protein localisation to cell tip, inhibition of protein localisation to cell tip, inhibition of protein localization to cell tip